{
  "term_label": "Unknown biological process",
  "term_id": "UNKNOWN:0002",
  "gene": "UniProtKB:Q8NGI8",
  "gene_name": "Olfactory receptor 5AN1",
  "gene_symbol": "OR5AN1"
}